{
  "gene": "UniProtKB:Q8NE65",
  "term_id": "GO:0005634",
  "gene_name": "Zinc finger protein 738",
  "gene_symbol": "ZNF738",
  "term_label": "nucleus"
}